TOR signaling [GO:0031929] (biological process) Definition: The series of molecular signals mediated by TOR (Target of rapamycin) proteins, members of the phosphoinositide (PI) 3-kinase related kinase (PIKK) family that act as serine/threonine kinases in response to nutrient availability or growth factors. Regulation: RO_0002211 by regulation of TOR signaling [GO:0032006]; negatively regulated by negative regulation of TOR signaling [GO:0032007]; positively regulated by positive regulation of TOR signaling [GO:0032008] Also known as: TOR signal transduction, TOR signaling pathway, TOR signalling pathway, target of rapamycin signaling pathway, target of rapamycin signalling pathway, TOR signaling cascade References: PMID:12372295 Subtypes: TORC1 signaling [GO:0038202], GO:0038203 Note: Note that this term should not be confused with 'torso signaling pathway ; GO:0008293', although torso is abbreviated 'tor'. Relationships: is a type of intracellular signal transduction [GO:0035556]